3-methylbutanal reductase [NAD(P)H] activity [GO:0046568] (molecular function) Definition: Catalysis of the reaction: 3-methylbutanol + NAD(P)+ = 3-methylbutanal + NAD(P)H + H+. 3-methylbutanal is also known as isovaleraldehyde. Also known as: 3-methylbutanol:NAD(P) oxidoreductase activity, 3-methylbutyraldehyde reductase activity, isoamyl alcohol oxidase activity, 3-methylbutanal reductase [NAD(P)] activity Sources: EC:1.1.1.265 Subtypes: 3-methylbutanal reductase (NADPH) activity [GO:0052675], 3-methylbutanal reductase (NADH) activity [GO:0052676] Relationships: is a type of alcohol dehydrogenase [NAD(P)+] activity [GO:0018455]